protein localization to eisosome filament [GO:0097446] (biological process) Definition: A process in which a protein is transported to, and/or maintained in, a specific location in a eisosome filament (also called linear eisosome), a filamentous cortical structure formed, in S. pombe, by the eisosome component Pil1. References: PMID:22869600, PMID:23722945 Sources: GOC:mah, GOC:vw Also known as: protein localization to linear eisosome Relationships: is a type of protein localization to cytoskeleton [GO:0044380]; is a type of protein localization to cell cortex [GO:0072697]